{
  "term_id": "GO:0000981",
  "gene_symbol": "ZNF506",
  "gene": "UniProtKB:Q5JVG8",
  "term_label": "DNA-binding transcription factor activity, RNA polymerase II-specific",
  "gene_name": "Zinc finger protein 506"
}